{
  "gene": "UniProtKB:Q969J3",
  "gene_symbol": "BORCS5",
  "term_id": "UNKNOWN:0001",
  "gene_name": "BLOC-1-related complex subunit 5",
  "term_label": "Unknown molecular function"
}